GMP biosynthetic process [GO:0006177] (biological process) Relationships: is a type of GO:0009152; is a type of purine ribonucleoside monophosphate biosynthetic process [GO:0009168]; is a type of GMP metabolic process [GO:0046037] Sources: ISBN:0198506732 Definition: The chemical reactions and pathways resulting in the formation of GMP, guanosine monophosphate. Subtypes: GO:0032263, 'de novo' GMP biosynthetic process [GO:0106387] Also known as: GMP anabolism, GMP biosynthesis, GMP formation, GMP synthesis